type 5 neuropeptide Y receptor binding [GO:0031845] (molecular function) Relationships: is a type of neuropeptide Y receptor binding [GO:0031841] Also known as: type 5 neuropeptide Y receptor ligand Definition: Binding to a type 5 neuropeptide Y receptor. Sources: GOC:mah, GOC:nln